{
  "term_label": "Unknown molecular function",
  "gene_symbol": "KIZ",
  "gene_name": "Centrosomal protein kizuna",
  "term_id": "UNKNOWN:0001",
  "gene": "UniProtKB:Q2M2Z5"
}